{
  "gene_symbol": "MRPL32",
  "gene": "UniProtKB:Q9BYC8",
  "term_label": "Unknown biological process",
  "gene_name": "Large ribosomal subunit protein bL32m",
  "term_id": "UNKNOWN:0002"
}